{
  "gene": "UniProtKB:Q6P4I2",
  "gene_symbol": "WDR73",
  "term_label": "cytoplasmic microtubule organization",
  "term_id": "GO:0031122",
  "gene_name": "WD repeat-containing protein 73"
}